{
  "gene": "UniProtKB:P51948",
  "term_id": "UNKNOWN:0001",
  "term_label": "Unknown molecular function",
  "gene_symbol": "MNAT1",
  "gene_name": "CDK-activating kinase assembly factor MAT1"
}